{
  "term_id": "GO:0005730",
  "gene": "UniProtKB:Q9BZI7",
  "term_label": "nucleolus",
  "gene_symbol": "UPF3B",
  "gene_name": "Regulator of nonsense transcripts 3B"
}